{
  "term_id": "UNKNOWN:0002",
  "term_label": "Unknown biological process",
  "gene_name": "Homologous recombination OB-fold protein",
  "gene": "UniProtKB:Q8N3J3",
  "gene_symbol": "HROB"
}